{
  "gene_symbol": "EHMT2",
  "term_id": "GO:0000785",
  "gene": "UniProtKB:Q96KQ7",
  "term_label": "chromatin",
  "gene_name": "Histone-lysine N-methyltransferase EHMT2"
}